{
  "term_id": "GO:0008046",
  "term_label": "axon guidance receptor activity",
  "gene_symbol": "HMCN2",
  "gene_name": "Hemicentin-2",
  "gene": "UniProtKB:Q8NDA2"
}